{
  "term_id": "UNKNOWN:0001",
  "gene": "UniProtKB:Q8IYE1",
  "gene_symbol": "CCDC13",
  "gene_name": "Coiled-coil domain-containing protein 13",
  "term_label": "Unknown molecular function"
}